{
  "gene": "UniProtKB:Q8TCJ2",
  "gene_symbol": "STT3B",
  "term_id": "GO:0043687",
  "term_label": "post-translational protein modification",
  "gene_name": "Dolichyl-diphosphooligosaccharide--protein glycosyltransferase subunit STT3B"
}